{
  "term_id": "GO:0030246",
  "gene_name": "C-type lectin domain family 4 member E",
  "gene_symbol": "CLEC4E",
  "gene": "UniProtKB:Q9ULY5",
  "term_label": "carbohydrate binding"
}